{
  "term_id": "GO:0005634",
  "gene": "UniProtKB:Q96MA1",
  "gene_name": "Doublesex- and mab-3-related transcription factor B1",
  "term_label": "nucleus",
  "gene_symbol": "DMRTB1"
}